vacuolar amino acid transmembrane transport [GO:0034487] (BP) Relationships: is a type of amino acid transmembrane transport [GO:0003333] Also known as: vacuolar amino acid membrane transport Sources: GOC:mah Note: Note that this term is not intended for use in annotating lateral movement within membranes. Definition: The process in which an amino acid is transported from one side of the vacuolar membrane to the other. Subtypes: basic amino acid transmembrane export from vacuole [GO:0034488], L-aspartate transmembrane export from vacuole [GO:0089703], aspartate transmembrane import into vacuole [GO:0090453]